{
  "gene_name": "Endoplasmic reticulum aminopeptidase 1",
  "gene_symbol": "ERAP1",
  "gene": "UniProtKB:Q9NZ08",
  "term_label": "proteolysis",
  "term_id": "GO:0006508"
}